{
  "gene_name": "Gamma-aminobutyric acid receptor-associated protein-like 2",
  "term_label": "mitophagy",
  "gene": "UniProtKB:P60520",
  "gene_symbol": "GABARAPL2",
  "term_id": "GO:0000423"
}